{
  "gene_symbol": "DUX4L4",
  "gene": "UniProtKB:P0CJ87",
  "gene_name": "Double homeobox protein 4-like protein 4",
  "term_id": "GO:0006357",
  "term_label": "regulation of transcription by RNA polymerase II"
}